{
  "term_label": "Unknown molecular function",
  "gene": "UniProtKB:Q9H497",
  "gene_symbol": "TOR3A",
  "term_id": "UNKNOWN:0001",
  "gene_name": "Torsin-3A"
}